regulation of intracellular transport [GO:0032386] (biological process) Definition: Any process that modulates the frequency, rate or extent of the directed movement of substances within cells. Sources: GOC:mah Relationships: is a type of regulation of transport [GO:0051049]; is a type of regulation of cellular localization [GO:0060341]; RO_0002211 intracellular transport [GO:0046907] Subtypes: regulation of intracellular lipid transport [GO:0032377], GO:0032387, positive regulation of intracellular transport [GO:0032388], GO:0032971, GO:0033157, regulation of nucleocytoplasmic transport [GO:0046822], regulation of ER to Golgi vesicle-mediated transport [GO:0060628], regulation of recycling endosome localization within postsynapse [GO:0099158], GO:1901301, GO:1902080, GO:1902513, regulation of early endosome to recycling endosome transport [GO:1902954], GO:1903335, regulation of dense core granule transport [GO:1904809], GO:1905279, GO:1905600, regulation of intraciliary anterograde transport [GO:1905796], regulation of intraciliary retrograde transport [GO:1905799], GO:2000641, regulation of retrograde axon cargo transport [GO:2001017], GO:2001135